{
  "gene_name": "Neurobeachin-like protein 1",
  "gene": "UniProtKB:Q6ZS30",
  "gene_symbol": "NBEAL1",
  "term_label": "cytosol",
  "term_id": "GO:0005829"
}